posterior lateral line neuromast hair cell differentiation [GO:0048923] (biological process) Sources: ISBN:0125296509 Relationships: is a type of neuromast hair cell differentiation [GO:0048886]; is part of GO:0048919 Definition: The process in which a relatively unspecialized cell acquires specialized features of a posterior lateral line neuromast hair cell. (N.B. This may be development of neuromast hair cell type or a set of cell of neuromast hair cell type. This will involve the change of a cell or set of cells from one cell identity to another). Hair cells are the sensory receptors of the neuromast and are located in a portion of the neuromast called the sensory strip. Each hair cell of the neuromast is morphologically polarized as a result of the relative position of the single kinocilium and the clusters of stereocilia on its apical surface. There are approximately seven hair cells within each neuromast, with each hair cell innervated by afferent and efferent neurons.